leaf formation [GO:0010338] (biological process) Regulation: regulated by regulation of leaf formation [GO:2000025] Definition: The process that gives rise to a leaf. This process pertains to the initial formation of a structure from unspecified parts. Relationships: is a type of plant organ development [GO:0099402]; is a type of plant organ formation [GO:1905393]; is part of GO:0009965 Sources: GOC:tair_curators